{
  "term_id": "UNKNOWN:0002",
  "gene_name": "CPX chromosomal region candidate gene 1 protein",
  "gene_symbol": "CPXCR1",
  "term_label": "Unknown biological process",
  "gene": "UniProtKB:Q8N123"
}